{
  "term_id": "GO:0007186",
  "gene_symbol": "GNRHR2",
  "gene_name": "Putative gonadotropin-releasing hormone II receptor",
  "term_label": "G protein-coupled receptor signaling pathway",
  "gene": "UniProtKB:Q96P88"
}